{
  "term_id": "GO:0007187",
  "gene_name": "5-hydroxytryptamine receptor 1D",
  "gene_symbol": "HTR1D",
  "gene": "UniProtKB:P28221",
  "term_label": "G protein-coupled receptor signaling pathway, coupled to cyclic nucleotide second messenger"
}